{
  "term_label": "synaptic vesicle budding from presynaptic endocytic zone membrane",
  "gene_name": "Dynamin-3",
  "term_id": "GO:0016185",
  "gene": "UniProtKB:Q9UQ16",
  "gene_symbol": "DNM3"
}